{
  "term_id": "GO:0034314",
  "gene": "UniProtKB:O15511",
  "term_label": "Arp2/3 complex-mediated actin nucleation",
  "gene_symbol": "ARPC5",
  "gene_name": "Actin-related protein 2_3 complex subunit 5"
}